{
  "term_id": "UNKNOWN:0002",
  "gene": "UniProtKB:Q86Y29",
  "gene_symbol": "BAGE3",
  "term_label": "Unknown biological process",
  "gene_name": "B melanoma antigen 3"
}